{
  "gene_name": "Immunoglobulin lambda joining 4 (non-functional) (Fragment)",
  "term_label": "Unknown molecular function",
  "gene": "UniProtKB:A0A0A0MTA1",
  "gene_symbol": "IGLJ4",
  "term_id": "UNKNOWN:0001"
}